cell adhesion involved in prostatic bud elongation [GO:0060519] (biological process) Relationships: is a type of cell adhesion [GO:0007155]; is part of primary prostatic bud elongation [GO:0060516] References: PMID:18977204 Sources: GOC:dph Definition: The attachment of a cell, either to another cell or to an underlying substrate such as the extracellular matrix, via cell adhesion molecules that contributes to the elongation of the primary prostatic bud.